{
  "gene_name": "Chromosome 6 open reading frame 48, isoform CRA_a",
  "term_id": "UNKNOWN:0001",
  "gene_symbol": "SNHG32",
  "term_label": "Unknown molecular function",
  "gene": "UniProtKB:A0A024RCN7"
}